regulation of xyloglucan catabolic process [GO:2000951] (BP) Also known as: regulation of xyloglucan catabolism Sources: GOC:mengo_curators Definition: Any process that modulates the frequency, rate or extent of xyloglucan catabolic process. Relationships: is a type of GO:2000988; regulates GO:2000899 Subtypes: negative regulation of xyloglucan catabolic process [GO:2000952], positive regulation of xyloglucan catabolic process [GO:2000953]